{
  "term_id": "UNKNOWN:0002",
  "gene": "UniProtKB:Q8WV48",
  "gene_name": "Coiled-coil domain-containing protein 107",
  "term_label": "Unknown biological process",
  "gene_symbol": "CCDC107"
}